acetate biosynthetic process [GO:0019413] (biological process) Sources: GOC:go_curators Subtypes: acetate biosynthetic process from carbon monoxide [GO:0019415] Also known as: acetate anabolism, acetate biosynthesis, acetate formation, acetate synthesis Relationships: is a type of GO:0006083; is a type of GO:0072330 Definition: The chemical reactions and pathways resulting in the formation of acetate, the anion of acetic acid.